{
  "term_id": "GO:0003828",
  "gene_name": "Alpha-N-acetylneuraminide alpha-2,8-sialyltransferase",
  "gene": "UniProtKB:Q92185",
  "term_label": "alpha-N-acetylneuraminate alpha-2,8-sialyltransferase activity",
  "gene_symbol": "ST8SIA1"
}